{
  "term_id": "UNKNOWN:0002",
  "gene_name": "Protein C19orf12",
  "gene": "UniProtKB:Q9NSK7",
  "gene_symbol": "C19orf12",
  "term_label": "Unknown biological process"
}